negative regulation of L-arginine import across plasma membrane [GO:1905542] (BP) References: PMID:14718525 Sources: GOC:TermGenie, GO_REF:0000058 Definition: Any process that stops, prevents or reduces the frequency, rate or extent of L-arginine import across plasma membrane. Relationships: is a type of negative regulation of organic acid transport [GO:0032891]; is_a negative regulation of transmembrane transport [GO:0034763]; is a type of negative regulation of amino acid transport [GO:0051956]; is_a regulation of L-arginine import across plasma membrane [GO:1905541]; negatively regulates L-arginine import across plasma membrane [GO:0097638] Also known as: down regulation of L-arginine import into cell, downregulation of L-arginine import into cell, negative regulation of L-arginine import into cell, inhibition of L-arginine import into cell